chorismate synthase activity [GO:0004107] (MF) Also known as: 5-O-(1-carboxyvinyl)-3-phosphoshikimate phosphate-lyase (chorismate-forming), 5-O-(1-carboxyvinyl)-3-phosphoshikimate phosphate-lyase activity, 5-enolpyruvylshikimate-3-phosphate phospholyase activity Sources: EC:4.2.3.5, RHEA:21020 Relationships: is a type of carbon-oxygen lyase activity, acting on phosphates [GO:0016838] Definition: Catalysis of the reaction: 5-O-(1-carboxyvinyl)-3-phosphoshikimate = chorismate + phosphate.